aspartate biosynthetic process [GO:0006532] (biological process) Relationships: is_a aspartate metabolic process [GO:0006531]; is a type of aspartate family amino acid biosynthetic process [GO:0009067]; is a type of dicarboxylic acid biosynthetic process [GO:0043650] Also known as: aspartate anabolism, aspartate biosynthesis, aspartate formation, aspartate synthesis Definition: The chemical reactions and pathways resulting in the formation of aspartate, the anion derived from aspartic acid, 2-aminobutanedioic acid. Sources: GOC:go_curators, ISBN:0198506732